eye pigment precursor transport [GO:0006856] (biological process) Sources: GOC:ai Definition: The directed movement of eye pigment precursors, the inactive forms of visual pigments, into, out of or within a cell, or between cells, by means of some agent such as a transporter or pore. Relationships: is a type of GO:0006810; is part of developmental pigmentation [GO:0048066]